{
  "term_label": "Unknown molecular function",
  "term_id": "UNKNOWN:0001",
  "gene_symbol": "PMS2P2",
  "gene": "UniProtKB:O95744",
  "gene_name": "Putative postmeiotic segregation increased 2-like protein 2"
}